positive regulation of protein localization to cell periphery [GO:1904377] (biological process) Definition: Any process that activates or increases the frequency, rate or extent of protein localization to cell periphery. References: PMID:18216290 Sources: GOC:TermGenie, GO_REF:0000058 Also known as: up regulation of protein localization to cell periphery, up-regulation of protein localization to cell periphery, upregulation of protein localization to cell periphery, activation of protein localization to cell periphery Relationships: is a type of positive regulation of protein localization [GO:1903829]; is a type of regulation of protein localization to cell periphery [GO:1904375]; positively regulates GO:1990778 Subtypes: positive regulation of protein localization to plasma membrane [GO:1903078], GO:1903569, positive regulation of protein localization to basolateral plasma membrane [GO:1904510], positive regulation of protein localization to cell cortex [GO:1904778]